glyoxysomal membrane [GO:0046861] (cellular component) Relationships: is_a GO:0005778; is part of GO:0009514 Also known as: glyoxysome membrane Sources: GOC:ai Definition: The lipid bilayer surrounding a glyoxysome.